'de novo' post-translational protein folding [GO:0051084] (BP) Definition: The process of assisting in the correct noncovalent folding of newly formed polypeptides or folding intermediates of polypeptides that have exited the ribosome and/or have been stabilized and transferred by other chaperone proteins. This process could involve several cycles of ATP hydrolysis. Relationships: is a type of 'de novo' protein folding [GO:0006458] Sources: GOC:rb Also known as: 'de novo' posttranslational protein folding